{
  "gene_name": "Dynein axonemal heavy chain 17",
  "gene": "UniProtKB:Q9UFH2",
  "term_id": "GO:0030286",
  "term_label": "dynein complex",
  "gene_symbol": "DNAH17"
}